brain-derived neurotrophic factor receptor activity [GO:0060175] (molecular function) Sources: GOC:bf, GOC:dph Definition: Combining with a brain-derived neurotrophic factor and transmitting the signal across the plasma membrane to initiate a change in cell activity. Relationships: is a type of transmembrane receptor protein tyrosine kinase activity [GO:0004714]; is a type of neurotrophin receptor activity [GO:0005030]; is part of brain-derived neurotrophic factor receptor signaling pathway [GO:0031547]; BFO_0000051 brain-derived neurotrophic factor binding [GO:0048403] Also known as: BDNF-activated receptor activity, brain-derived neurotrophic factor-activated receptor activity, BDNF receptor activity Note: Note that this term represents an activity and not a gene product, and should only be used when the receptor binds the ligand BDNF. For receptors that bind other growth factors, consider annotating to other terms under 'transmembrane signaling receptor activity ; GO:0004888.